{
  "gene_symbol": "NRIP2",
  "gene": "UniProtKB:Q9BQI9",
  "gene_name": "Nuclear receptor-interacting protein 2",
  "term_id": "GO:0006508",
  "term_label": "proteolysis"
}